tRNA-4-demethylwyosine synthase activity [GO:0102521] (molecular function) Relationships: is a type of oxo-acid-lyase activity [GO:0016833]; is a type of catalytic activity, acting on a tRNA [GO:0140101] Definition: Catalysis of the reaction: pyruvate + S-adenosyl-L-methionine + N1-methylguanine37 in tRNAPhe = L-methionine + 5'-deoxyadenosine + carbon dioxide + H2O + 4-demethylwyosine37 in tRNAPhe. References: PMID:34184886 Sources: GOC:pz, RHEA:36347